{
  "term_label": "Unknown biological process",
  "gene_symbol": "PLCXD3",
  "gene_name": "PI-PLC X domain-containing protein 3",
  "term_id": "UNKNOWN:0002",
  "gene": "UniProtKB:Q63HM9"
}